regulation of ferroptosis [GO:0110075] (biological process) Subtypes: GO:0110076, positive regulation of ferroptosis [GO:0160020] Relationships: is a type of regulation of programmed cell death [GO:0043067]; regulates ferroptosis [GO:0097707] Definition: Any process that modulates the frequency, rate or extent of ferroptosis. References: PMID:24439385, PMID:25402683, PMID:29290465 Sources: GOC:sp